blood vessel lumenization [GO:0072554] (biological process) Subtypes: blood vessel lumen ensheathment [GO:0097496] Relationships: is_a endothelial tube morphogenesis [GO:0061154]; is part of blood vessel morphogenesis [GO:0048514] References: PMID:16799567, PMID:20926893 Sources: GOC:dsf Definition: The process in which a developing blood vessel forms an endothelial lumen through which blood will flow.